{
  "gene": "UniProtKB:Q68BL8",
  "term_label": "extracellular space",
  "gene_name": "Olfactomedin-like protein 2B",
  "term_id": "GO:0005615",
  "gene_symbol": "OLFML2B"
}